{
  "term_id": "GO:0007052",
  "term_label": "mitotic spindle organization",
  "gene": "UniProtKB:Q15468",
  "gene_name": "SCL-interrupting locus protein",
  "gene_symbol": "STIL"
}